{
  "gene_symbol": "CRY2",
  "gene_name": "Cryptochrome-2",
  "term_label": "cytoplasm",
  "term_id": "GO:0005737",
  "gene": "UniProtKB:Q49AN0"
}